galacturonokinase activity [GO:0047912] (molecular function) Relationships: is a type of GO:0016301; is_a phosphotransferase activity, alcohol group as acceptor [GO:0016773] Also known as: ATP:D-galacturonate 1-phosphotransferase activity, galacturonokinase (phosphorylating) D-galacturonic acid kinase activity Definition: Catalysis of the reaction: alpha-D-galacturonate + ATP = 1-phospho-alpha-D-galacturonate + ADP + 2 H+. Sources: EC:2.7.1.44, RHEA:12965